{
  "gene": "UniProtKB:P08217",
  "gene_symbol": "CELA2A",
  "gene_name": "Chymotrypsin-like elastase family member 2A",
  "term_label": "regulation of platelet aggregation",
  "term_id": "GO:0090330"
}